indole phytoalexin catabolic process [GO:0046216] (biological process) Definition: The chemical reactions and pathways resulting in the breakdown of indole phytoalexins, any indole compound produced by plants as part of their defense response. Sources: GOC:ai Also known as: indole phytoalexin breakdown, indole phytoalexin catabolism, indole phytoalexin degradation Relationships: is a type of indole-containing compound catabolic process [GO:0042436]; is a type of detoxification of nitrogen compound [GO:0051410]; is a type of phytoalexin catabolic process [GO:0052316]